regulation of follicle cell microvillus organization [GO:0032531] (biological process) Relationships: is a type of regulation of microvillus organization [GO:0032530]; regulates follicle cell microvillus organization [GO:0032529] Subtypes: regulation of follicle cell microvillus length [GO:0032533] Definition: Any process that modulates the frequency, rate or extent of a process involved in the formation, arrangement of constituent parts, or disassembly of a microvillus on a follicle cell. Also known as: regulation of follicle cell microvillus organisation, regulation of follicle cell microvillus organization and biogenesis Sources: GOC:mah